{
  "gene_symbol": "CSRP3",
  "gene": "UniProtKB:P50461",
  "term_id": "GO:0060537",
  "gene_name": "Cysteine and glycine-rich protein 3",
  "term_label": "muscle tissue development"
}